{
  "term_label": "Unknown cellular component",
  "term_id": "UNKNOWN:0003",
  "gene": "UniProtKB:Q05655",
  "gene_symbol": "PRKCD",
  "gene_name": "Protein kinase C delta type"
}